{
  "gene_symbol": "RPUSD4",
  "gene_name": "Pseudouridylate synthase RPUSD4, mitochondrial",
  "term_label": "Unknown cellular component",
  "term_id": "UNKNOWN:0003",
  "gene": "UniProtKB:Q96CM3"
}